{
  "term_id": "GO:0016616",
  "gene_name": "Short-chain dehydrogenase_reductase family 42E member 1",
  "gene": "UniProtKB:Q8WUS8",
  "gene_symbol": "SDR42E1",
  "term_label": "oxidoreductase activity, acting on the CH-OH group of donors, NAD or NADP as acceptor"
}